positive regulation of synaptic transmission, GABAergic [GO:0032230] (biological process) Also known as: up regulation of synaptic transmission, GABAergic, up-regulation of synaptic transmission, GABAergic, upregulation of synaptic transmission, GABAergic, activation of synaptic transmission, GABAergic, stimulation of synaptic transmission, GABAergic Definition: Any process that activates, maintains or increases the frequency, rate or extent of GABAergic synaptic transmission, the process of communication from a neuron to another neuron across a synapse using the neurotransmitter gamma-aminobutyric acid (GABA). Sources: GOC:mah Relationships: is a type of regulation of synaptic transmission, GABAergic [GO:0032228]; is a type of positive regulation of synaptic transmission [GO:0050806]; positively regulates synaptic transmission, GABAergic [GO:0051932]